{
  "term_id": "UNKNOWN:0002",
  "gene_name": "Olfactory receptor",
  "gene_symbol": "OR2A1",
  "gene": "UniProtKB:A0A2R8YEG4",
  "term_label": "Unknown biological process"
}